{
  "gene_symbol": "DPM3",
  "gene": "UniProtKB:Q9P2X0",
  "term_label": "Unknown biological process",
  "gene_name": "Dolichol-phosphate mannosyltransferase subunit 3",
  "term_id": "UNKNOWN:0002"
}